{
  "term_label": "Unknown cellular component",
  "term_id": "UNKNOWN:0003",
  "gene": "UniProtKB:O15428",
  "gene_name": "Putative PIN1-like protein",
  "gene_symbol": "PIN1P1"
}